{
  "gene_name": "SH3 and PX domain-containing protein 2B",
  "term_label": "superoxide anion generation",
  "term_id": "GO:0042554",
  "gene": "UniProtKB:A1X283",
  "gene_symbol": "SH3PXD2B"
}